protein localization to nucleus [GO:0034504] (biological process) Definition: A process in which a protein transports or maintains the localization of another protein to the nucleus. Sources: GOC:ecd Also known as: protein localisation to nucleus, protein localization in cell nucleus, protein localization in nucleus, protein targeting to nucleus Relationships: is a type of protein localization to organelle [GO:0033365] Subtypes: GO:0006606, protein localization to nuclear envelope [GO:0090435], protein localization to Mei2 nuclear dot [GO:1902549], GO:1902570, protein localization to condensed nuclear chromosome [GO:1903084], protein localization to nuclear periphery [GO:1990139], GO:1990173 Regulation: regulated by regulation of protein localization to nucleus [GO:1900180]; negatively regulated by negative regulation of protein localization to nucleus [GO:1900181]; positively regulated by positive regulation of protein localization to nucleus [GO:1900182]